{
  "term_label": "protein C-terminal S-isoprenylcysteine carboxyl O-methyltransferase activity",
  "gene_symbol": "ICMT",
  "gene": "UniProtKB:O60725",
  "gene_name": "Protein-S-isoprenylcysteine O-methyltransferase",
  "term_id": "GO:0004671"
}